{
  "gene": "UniProtKB:Q96PF1",
  "gene_symbol": "TGM7",
  "gene_name": "Protein-glutamine gamma-glutamyltransferase Z",
  "term_label": "Unknown cellular component",
  "term_id": "UNKNOWN:0003"
}